regulation of interleukin-27 production [GO:0032671] (biological process) Also known as: regulation of IL-27 production, regulation of interleukin-27 biosynthetic process, regulation of interleukin-27 formation, regulation of interleukin-27 synthesis Definition: Any process that modulates the frequency, rate, or extent of interleukin-27 production. Relationships: is a type of GO:0001817; regulates GO:0032631 Subtypes: negative regulation of interleukin-27 production [GO:0032711], positive regulation of interleukin-27 production [GO:0032751] Sources: GOC:mah